{
  "gene_name": "Protein PPP4R3C",
  "gene": "UniProtKB:Q6ZMV5",
  "term_label": "regulation of double-strand break repair",
  "term_id": "GO:2000779",
  "gene_symbol": "PPP4R3C"
}